{
  "gene": "UniProtKB:Q6ZN92",
  "term_label": "magnesium ion binding",
  "gene_symbol": "Q6ZN92",
  "gene_name": "Putative inactive deoxyuridine 5'-triphosphate nucleotidohydrolase-like protein FLJ16323",
  "term_id": "GO:0000287"
}